tube morphogenesis [GO:0035239] (biological process) Relationships: is a type of anatomical structure morphogenesis [GO:0009653]; is part of tube development [GO:0035295] References: PMID:14624839 Sources: GOC:bf Subtypes: GO:0007426, tube fusion [GO:0035146], GO:0035848, GO:0048514, GO:0048546, semicircular canal morphogenesis [GO:0048752], branching morphogenesis of an epithelial tube [GO:0048754], cloacal septation [GO:0060197], bronchus morphogenesis [GO:0060434], bronchiole morphogenesis [GO:0060436], epithelial tube morphogenesis [GO:0060562], ureter morphogenesis [GO:0072197] Definition: The process in which the anatomical structures of a tube are generated and organized. Epithelial and endothelial tubes transport gases, liquids and cells from one site to another and form the basic structure of many organs and tissues, with tube shape and organization varying from the single-celled excretory organ in Caenorhabditis elegans to the branching trees of the mammalian kidney and insect tracheal system.